{
  "gene_name": "Myeloid-derived growth factor",
  "term_label": "positive regulation of angiogenesis",
  "term_id": "GO:0045766",
  "gene": "UniProtKB:Q969H8",
  "gene_symbol": "MYDGF"
}